{
  "term_label": "arginine-tRNA ligase activity",
  "gene_symbol": "RARS2",
  "term_id": "GO:0004814",
  "gene": "UniProtKB:Q5T160",
  "gene_name": "Probable arginine--tRNA ligase, mitochondrial"
}